{
  "term_label": "RNA polymerase II transcription regulatory region sequence-specific DNA binding",
  "gene_name": "Putative zinc finger protein 705EP",
  "gene_symbol": "ZNF705EP",
  "term_id": "GO:0000977",
  "gene": "UniProtKB:A8MWA4"
}